{
  "gene": "UniProtKB:Q01459",
  "term_id": "GO:0006032",
  "gene_symbol": "CTBS",
  "gene_name": "Di-N-acetylchitobiase",
  "term_label": "chitin catabolic process"
}